positive regulation of nuclear migration during mitotic telophase [GO:1902854] (BP) Definition: Any process that activates or increases the frequency, rate or extent of nuclear migration during mitotic telophase. References: PMID:23087209 Sources: GOC:TermGenie, GO_REF:0000058 Also known as: up regulation of nuclear migration during mitotic telophase, up-regulation of nuclear migration during mitotic telophase, upregulation of nuclear migration during mitotic telophase, activation of nuclear migration during mitotic telophase Relationships: is a type of positive regulation of nuclear migration along microtubule [GO:1902840]; is a type of GO:1902852; positively regulates nuclear migration during mitotic telophase [GO:0090561]